{
  "gene_name": "Hexokinase-4",
  "gene": "UniProtKB:P35557",
  "term_id": "GO:0001678",
  "gene_symbol": "GCK",
  "term_label": "intracellular glucose homeostasis"
}